{
  "term_label": "Unknown cellular component",
  "gene_symbol": "TCP11L2",
  "term_id": "UNKNOWN:0003",
  "gene": "UniProtKB:Q8N4U5",
  "gene_name": "T-complex protein 11-like protein 2"
}